spinal cord patterning [GO:0021511] (biological process) Relationships: is a type of regionalization [GO:0003002]; is part of spinal cord development [GO:0021510] Definition: The regionalization process that regulates the coordinated growth and establishes the non-random spatial arrangement of the spinal cord. Sources: GOC:cls, GOC:dgh, GOC:dph, GOC:jid, GO_REF:0000021